alpha,alpha-trehalose-phosphate synthase (GDP-forming) activity [GO:0047260] (molecular function) Definition: Catalysis of the reaction: GDP-D-glucose + glucose-6-phosphate = alpha,alpha-trehalose 6-phosphate + GDP. Sources: EC:2.4.1.36, MetaCyc:2.4.1.36-RXN Also known as: GDP-glucose-glucosephosphate glucosyltransferase activity, GDP-glucose:D-glucose-6-phosphate 1-alpha-D-glucosyltransferase activity, GDPglucose-glucose-phosphate glucosyltransferase activity, GDPglucose:D-glucose-6-phosphate 1-alpha-D-glucosyltransferase activity, guanosine diphosphoglucose-glucose phosphate glucosyltransferase activity, trehalose phosphate synthase (GDP-forming) activity Relationships: is_a hexosyltransferase activity [GO:0016758]